{
  "gene": "UniProtKB:Q15431",
  "gene_symbol": "SYCP1",
  "term_id": "GO:0000801",
  "gene_name": "Synaptonemal complex protein 1",
  "term_label": "central element"
}